response to odorant [GO:1990834] (biological process) Definition: Any process that results in a change in state or activity of a cell or an organism (in terms of movement, secretion, enzyme production, gene expression, etc.) as a result of an odorant stimulus. An odorant is any substance capable of stimulating the sense of smell. References: PMID:11268007 Relationships: is a type of GO:0042221